{
  "gene_name": "Centromere-associated protein E",
  "term_label": "mitotic cell cycle",
  "gene": "UniProtKB:Q02224",
  "gene_symbol": "CENPE",
  "term_id": "GO:0000278"
}